{
  "term_id": "GO:0005886",
  "term_label": "plasma membrane",
  "gene_symbol": "TSPAN19",
  "gene_name": "Tetraspanin-19",
  "gene": "UniProtKB:P0C672"
}